alpha-N-acetylneuraminate alpha-2,8-sialyltransferase activity [GO:0003828] (molecular function) Also known as: alpha-N-acetylneuraminide alpha-2,8-sialyltransferase activity, alpha-2,8-sialyltransferase activity, cytidine monophosphoacetylneuraminate-ganglioside GM3, ganglioside GD3 synthase activity, ganglioside GD3 synthetase sialyltransferase activity Sources: EC:2.4.3.8 Definition: Catalysis of the reaction: CMP-N-acetylneuraminate + alpha-N-acetylneuraminyl-(2->3)-beta-D-galactosyl-R = CMP + alpha-N-acetylneuraminyl-(2->8)-alpha-N-acetylneuraminyl-(2->3)-beta-D-galactosyl-R. Relationships: is a type of sialyltransferase activity [GO:0008373]